{
  "gene_symbol": "AMN",
  "gene_name": "Protein amnionless",
  "term_id": "GO:0006898",
  "term_label": "receptor-mediated endocytosis",
  "gene": "UniProtKB:Q9BXJ7"
}